{
  "term_label": "cytoplasm",
  "gene_symbol": "SULT1A1",
  "term_id": "GO:0005737",
  "gene": "UniProtKB:P50225",
  "gene_name": "Sulfotransferase 1A1"
}